{
  "gene_name": "NADH dehydrogenase (ubiquinone) complex I, assembly factor 6",
  "gene_symbol": "NDUFAF6",
  "gene": "UniProtKB:Q330K2",
  "term_id": "GO:0032981",
  "term_label": "mitochondrial respiratory chain complex I assembly"
}